{
  "gene_symbol": "PSORS1C2",
  "term_label": "Unknown biological process",
  "term_id": "UNKNOWN:0002",
  "gene_name": "Psoriasis susceptibility 1 candidate gene 2 protein",
  "gene": "UniProtKB:Q9UIG4"
}